{
  "gene": "UniProtKB:Q9UFF9",
  "term_id": "GO:0000932",
  "term_label": "P-body",
  "gene_symbol": "CNOT8",
  "gene_name": "CCR4-NOT transcription complex subunit 8"
}